{
  "term_label": "structural constituent of ribosome",
  "gene_symbol": "ISG15",
  "gene_name": "Ubiquitin-like protein ISG15",
  "term_id": "GO:0003735",
  "gene": "UniProtKB:P05161"
}